{
  "gene_symbol": "NR1H2",
  "gene_name": "Oxysterols receptor LXR-beta",
  "gene": "UniProtKB:P55055",
  "term_id": "GO:0000122",
  "term_label": "negative regulation of transcription by RNA polymerase II"
}